{
  "gene": "UniProtKB:Q13572",
  "gene_symbol": "ITPK1",
  "term_label": "Unknown biological process",
  "term_id": "UNKNOWN:0002",
  "gene_name": "Inositol-tetrakisphosphate 1-kinase"
}